microtubule nucleator activity [GO:0140490] (molecular function) Definition: The action of a molecule that provides a shape mimicking the end of a microtubule to seed the formation of a new microtubule via self-assembly. Also known as: microtubule nucleation template activity References: PMID:20631709, PMID:21993292 Relationships: is a type of GO:0140489